{
  "gene_name": "Gastrin",
  "term_id": "GO:0005179",
  "gene_symbol": "GAST",
  "term_label": "hormone activity",
  "gene": "UniProtKB:P01350"
}